{
  "gene_name": "Kinesin-like protein KIF28P",
  "term_label": "cytoplasm",
  "gene_symbol": "KIF28P",
  "term_id": "GO:0005737",
  "gene": "UniProtKB:B7ZC32"
}